{
  "term_id": "GO:0005790",
  "gene_symbol": "RYR3",
  "gene": "UniProtKB:Q15413",
  "gene_name": "Ryanodine receptor 3",
  "term_label": "smooth endoplasmic reticulum"
}